auditory receptor cell stereocilium organization [GO:0060088] (biological process) Relationships: is a type of GO:0060122; is part of GO:0002093 Also known as: auditory receptor cell stereocilium organisation, auditory receptor cell stereocilium organization and biogenesis Definition: A process that is carried out at the cellular level which results in the assembly, arrangement of constituent parts, or disassembly of a stereocilium. A stereocilium is an actin-based protrusion from the apical surface of auditory hair cells. References: PMID:10978835 Sources: GOC:dph